polyamine biosynthetic process [GO:0006596] (BP) Relationships: is a type of polyamine metabolic process [GO:0006595]; is a type of biogenic amine biosynthetic process [GO:0042401] Regulation: regulated by regulation of polyamine biosynthetic process [GO:0010967]; negatively regulated by negative regulation of polyamine biosynthetic process [GO:0170066] Subtypes: spermine biosynthetic process [GO:0006597], spermidine biosynthetic process [GO:0008295], putrescine biosynthetic process [GO:0009446], GO:0045312, trimethylenediamine biosynthetic process [GO:1901057], GO:1903603 Definition: The chemical reactions and pathways resulting in the formation of polyamines, any organic compound containing two or more amino groups. Sources: ISBN:0198506732 Also known as: polyamine anabolism, polyamine biosynthesis, polyamine formation, polyamine synthesis